UDP-beta-L-arabinofuranose transporter activity [GO:0140819] (molecular function) Relationships: is a type of pyrimidine nucleotide-sugar transmembrane transporter activity [GO:0015165] Definition: Enables the transfer of UDP-beta-L-arabinofuranose from one side of a membrane to the other. References: PMID:28373556